phosphate:acyl-[acyl carrier protein] acyltransferase activity [GO:0043811] (molecular function) Relationships: is a type of GO:0016747 Definition: Catalysis of the reaction: a fatty acyl-[acyl-carrier protein] + orthophosphate = acyl phosphate + [acyl-carrier protein]. Sources: RHEA:42292